{
  "term_label": "Unknown biological process",
  "gene": "UniProtKB:O94967",
  "term_id": "UNKNOWN:0002",
  "gene_symbol": "WDR47",
  "gene_name": "WD repeat-containing protein 47"
}